{
  "gene": "UniProtKB:Q5MCW4",
  "term_id": "GO:0000981",
  "term_label": "DNA-binding transcription factor activity, RNA polymerase II-specific",
  "gene_name": "Zinc finger protein 569",
  "gene_symbol": "ZNF569"
}